4-amino-4-deoxy-alpha-L-arabinopyranosyl undecaprenyl phosphate biosynthetic process [GO:0036108] (biological process) Definition: The chemical reactions and pathways resulting in the formation of 4-amino-4-deoxy-alpha-L-arabinopyranosyl undecaprenyl phosphate, a precursor of 4-amino-4-deoxy-L-arabinose (L-Ara4N). Also known as: 4-amino-4-deoxy-alpha-L-arabinopyranosyl undecaprenyl phosphate anabolism, 4-amino-4-deoxy-alpha-L-arabinopyranosyl undecaprenyl phosphate biosynthesis, 4-amino-4-deoxy-alpha-L-arabinopyranosyl undecaprenyl phosphate formation, 4-amino-4-deoxy-alpha-L-arabinopyranosyl undecaprenyl phosphate synthesis, undecaprenyl phosphate alpha-L-Ara4N biosynthesis References: PMID:15695810 Sources: GOC:yaf Relationships: is a type of phospholipid biosynthetic process [GO:0008654]; is a type of glycolipid biosynthetic process [GO:0009247]; is a type of terpenoid biosynthetic process [GO:0016114]